negative regulation of cellular response to vascular endothelial growth factor stimulus [GO:1902548] (biological process) References: PMID:17895370 Sources: GOC:BHF, GOC:TermGenie, GOC:rl Also known as: down regulation of cellular response to VEGF, down regulation of cellular response to vascular endothelial growth factor, down regulation of cellular response to vascular endothelial growth factor stimulus, down-regulation of cellular response to VEGF, down-regulation of cellular response to vascular endothelial growth factor, down-regulation of cellular response to vascular endothelial growth factor stimulus, downregulation of cellular response to VEGF, downregulation of cellular response to vascular endothelial growth factor, downregulation of cellular response to vascular endothelial growth factor stimulus, negative regulation of cellular response to VEGF, negative regulation of cellular response to vascular endothelial growth factor, down regulation of cellular response to VEGFA, down regulation of cellular response to VEGFB, down-regulation of cellular response to VEGFA, down-regulation of cellular response to VEGFB, downregulation of cellular response to VEGFA, downregulation of cellular response to VEGFB, inhibition of cellular response to VEGF, inhibition of cellular response to VEGFA, inhibition of cellular response to VEGFB, inhibition of cellular response to vascular endothelial growth factor, inhibition of cellular response to vascular endothelial growth factor stimulus, negative regulation of cellular response to VEGFA, negative regulation of cellular response to VEGFB Relationships: is a type of GO:0090288; is a type of regulation of cellular response to vascular endothelial growth factor stimulus [GO:1902547]; RO_0002212 cellular response to vascular endothelial growth factor stimulus [GO:0035924] Subtypes: negative regulation of vascular endothelial growth factor signaling pathway [GO:1900747], negative regulation of endothelial cell chemotaxis to vascular endothelial growth factor [GO:1904858] Definition: Any process that stops, prevents or reduces the frequency, rate or extent of cellular response to vascular endothelial growth factor stimulus. Note: ADAMTS12 (UniProt ID P58397) in human in PMID:17895370 inhibits the formation of VEGF-induced tubular structures in BAE-1 cells (endothelial cell line).